{
  "term_label": "plasma membrane",
  "gene_name": "NALCN channel auxiliary factor 2",
  "gene_symbol": "NALF2",
  "term_id": "GO:0005886",
  "gene": "UniProtKB:O75949"
}